{
  "gene_name": "Humanin-like 10",
  "gene_symbol": "MTRNR2L10",
  "term_id": "UNKNOWN:0003",
  "gene": "UniProtKB:P0CJ77",
  "term_label": "Unknown cellular component"
}